negative regulation of calcium ion transport into cytosol [GO:0010523] (biological process) Sources: GOC:dph, GOC:tb Relationships: is a type of GO:0010522; is a type of negative regulation of cytosolic calcium ion concentration [GO:0051481]; is a type of negative regulation of calcium ion transmembrane transport [GO:1903170]; negatively regulates GO:0060402 Definition: Any process that decreases the rate of the directed movement of calcium ions into the cytosol of a cell. The cytosol is that part of the cytoplasm that does not contain membranous or particulate subcellular components. Subtypes: negative regulation of calcium ion transport into cytosol involved in cellular response to salt stress [GO:1901200]